{
  "gene_name": "Exosome complex component RRP40",
  "gene": "UniProtKB:Q9NQT5",
  "term_id": "GO:0071038",
  "gene_symbol": "EXOSC3",
  "term_label": "TRAMP-dependent tRNA surveillance pathway"
}